{
  "gene_name": "Septin-10",
  "gene_symbol": "SEPTIN10",
  "term_label": "cytoskeleton-dependent cytokinesis",
  "term_id": "GO:0061640",
  "gene": "UniProtKB:Q9P0V9"
}